{
  "term_label": "Unknown cellular component",
  "gene_symbol": "FOXI2",
  "term_id": "UNKNOWN:0003",
  "gene": "UniProtKB:Q6ZQN5",
  "gene_name": "Forkhead box protein I2"
}